negative regulation of syringal lignin biosynthetic process [GO:1901429] (biological process) Definition: Any process that stops, prevents or reduces the frequency, rate or extent of syringal lignin biosynthetic process. Sources: GOC:TermGenie Relationships: is a type of negative regulation of secondary metabolite biosynthetic process [GO:1900377]; is_a regulation of syringal lignin biosynthetic process [GO:1901428]; negatively regulates syringal lignin biosynthetic process [GO:1901066] Also known as: down regulation of S-lignin biosynthetic process, down regulation of syringal lignin anabolism, down regulation of syringal lignin biosynthesis, down regulation of syringal lignin biosynthetic process, down regulation of syringal lignin formation, down regulation of syringal lignin synthesis, down-regulation of S-lignin biosynthetic process, down-regulation of syringal lignin anabolism, down-regulation of syringal lignin biosynthesis, down-regulation of syringal lignin biosynthetic process, down-regulation of syringal lignin formation, down-regulation of syringal lignin synthesis, downregulation of S-lignin biosynthetic process, downregulation of syringal lignin anabolism, downregulation of syringal lignin biosynthesis, downregulation of syringal lignin biosynthetic process, downregulation of syringal lignin formation, downregulation of syringal lignin synthesis, inhibition of S-lignin biosynthetic process, inhibition of syringal lignin anabolism, inhibition of syringal lignin biosynthesis, inhibition of syringal lignin formation, inhibition of syringal lignin synthesis, negative regulation of S-lignin biosynthetic process, negative regulation of syringal lignin anabolism, negative regulation of syringal lignin biosynthesis, negative regulation of syringal lignin formation, negative regulation of syringal lignin synthesis, inhibition of syringal lignin biosynthetic process